{
  "term_label": "Unknown molecular function",
  "term_id": "UNKNOWN:0001",
  "gene": "UniProtKB:Q5T0U0",
  "gene_name": "Coiled-coil domain-containing protein 122",
  "gene_symbol": "CCDC122"
}